interferon-delta production [GO:0072645] (biological process) Definition: The appearance of interferon-delta due to biosynthesis or secretion following a cellular stimulus, resulting in an increase in its intracellular or extracellular levels. Relationships: is a type of type I interferon production [GO:0032606] Note: Note that this term is in the subset of terms that should not be used for direct gene product annotation. Instead, select one of the 'regulation' children terms. Also known as: IFN-delta production, IFND production, interferon-delta secretion References: PMID:15546383 Sources: GOC:BHF, GOC:mah